{
  "term_label": "Unknown cellular component",
  "gene_name": "Protein kinase C theta type",
  "term_id": "UNKNOWN:0003",
  "gene_symbol": "PRKCQ",
  "gene": "UniProtKB:Q04759"
}